response to chondroitin 6'-sulfate [GO:1905439] (biological process) Relationships: is a type of response to nitrogen compound [GO:1901698]; is a type of GO:1901700 References: PMID:22365850 Sources: GOC:TermGenie, GO_REF:0000071 Subtypes: cellular response to chondroitin 6'-sulfate [GO:1905440] Definition: Any process that results in a change in state or activity of a cell or an organism (in terms of movement, secretion, enzyme production, gene expression, etc.) as a result of a chondroitin 6'-sulfate stimulus.